{
  "gene": "UniProtKB:Q14957",
  "gene_symbol": "GRIN2C",
  "gene_name": "Glutamate receptor ionotropic, NMDA 2C",
  "term_id": "GO:1904315",
  "term_label": "transmitter-gated monoatomic ion channel activity involved in regulation of postsynaptic membrane potential"
}